{
  "term_id": "GO:0000423",
  "gene": "UniProtKB:Q5VWJ9",
  "gene_name": "Sorting nexin-30",
  "term_label": "mitophagy",
  "gene_symbol": "SNX30"
}